{
  "term_label": "sphingolipid biosynthetic process",
  "gene_symbol": "HACD2",
  "gene_name": "Very-long-chain (3R)-3-hydroxyacyl-CoA dehydratase 2",
  "gene": "UniProtKB:Q6Y1H2",
  "term_id": "GO:0030148"
}